{
  "gene_name": "Adhesion G protein-coupled receptor A2",
  "term_id": "GO:0005886",
  "gene": "UniProtKB:Q96PE1",
  "term_label": "plasma membrane",
  "gene_symbol": "ADGRA2"
}